{
  "term_id": "GO:0005783",
  "gene_name": "1-acyl-sn-glycerol-3-phosphate acyltransferase epsilon",
  "term_label": "endoplasmic reticulum",
  "gene": "UniProtKB:Q9NUQ2",
  "gene_symbol": "AGPAT5"
}